chondrocyte development involved in endochondral bone morphogenesis [GO:0003433] (biological process) Definition: The progression of a chondrocyte over time from after its commitment to its mature state where the chondrocyte will contribute to the shaping of an endochondral bone. Sources: GOC:ascb_2009, GOC:dph, GOC:tb Relationships: is a type of GO:0002063; is part of chondrocyte differentiation involved in endochondral bone morphogenesis [GO:0003413] Subtypes: growth plate cartilage chondrocyte development [GO:0003431]